{
  "term_id": "GO:0003727",
  "gene": "UniProtKB:Q8IY21",
  "term_label": "single-stranded RNA binding",
  "gene_symbol": "DDX60",
  "gene_name": "Probable ATP-dependent RNA helicase DDX60"
}